plasmodesma organization [GO:0009663] (biological process) Also known as: plasmodesma organisation, plasmodesma organization and biogenesis, plasmodesmata organization and biogenesis Relationships: is a type of cell-cell junction organization [GO:0045216] Definition: A process that is carried out at the cellular level which results in the assembly, arrangement of constituent parts, or disassembly of a plasmodesma, a fine cytoplasmic channel, found in all higher plants, that connects the cytoplasm of one cell to that of an adjacent cell. References: PMID:29880547 Sources: GOC:mah